{
  "gene_name": "Alpha-2-macroglobulin",
  "gene": "UniProtKB:P01023",
  "term_id": "GO:0005615",
  "gene_symbol": "A2M",
  "term_label": "extracellular space"
}